transcription factor TFTC complex [GO:0033276] (cellular component) Relationships: is a type of SAGA-type complex [GO:0070461]; is a type of RNA polymerase II transcription regulator complex [GO:0090575]; BFO_0000050 RNA polymerase II, holoenzyme [GO:0016591] References: PMID:10373431, PMID:9603525 Definition: A protein complex that does not contain either a TATA-binding protein (TBP) or a TBP-like factor, but is composed of several TAFIIs and other proteins, including a histone acetyltransferase. This complex is able to nucleate transcription initiation by RNA polymerase II, can mediate transcriptional activation, and has histone acetyltransferase activity.